pollen tube guidance [GO:0010183] (BP) Definition: The process in which the growth of pollen tube is directed towards the female gametophyte. Relationships: is a type of positive chemotaxis [GO:0050918]; is part of pollen tube development [GO:0048868] Regulation: negatively regulated by negative regulation of pollen tube guidance [GO:0160068] Sources: GOC:lr